{
  "term_label": "MHC class II protein complex binding",
  "term_id": "GO:0023026",
  "gene_name": "HLA class II histocompatibility antigen, DQ alpha 1 chain",
  "gene_symbol": "HLA-DQA1",
  "gene": "UniProtKB:P01909"
}